{
  "term_label": "basolateral plasma membrane",
  "gene_name": "FERM and PDZ domain-containing protein 2",
  "gene": "UniProtKB:Q68DX3",
  "term_id": "GO:0016323",
  "gene_symbol": "FRMPD2"
}